{
  "term_id": "GO:0007346",
  "gene_name": "Cyclin-dependent kinases regulatory subunit 1",
  "gene": "UniProtKB:P61024",
  "gene_symbol": "CKS1B",
  "term_label": "regulation of mitotic cell cycle"
}